{
  "term_label": "serotonin:sodium:chloride symporter activity",
  "gene_symbol": "SLC18A1",
  "term_id": "GO:0005335",
  "gene_name": "Chromaffin granule amine transporter",
  "gene": "UniProtKB:P54219"
}